{
  "gene_name": "Apolipoprotein E",
  "gene_symbol": "APOE",
  "term_label": "phosphatidylcholine-sterol O-acyltransferase activator activity",
  "term_id": "GO:0060228",
  "gene": "UniProtKB:P02649"
}